{
  "term_id": "GO:0007088",
  "gene": "UniProtKB:Q9H0W5",
  "gene_name": "Coiled-coil domain-containing protein 8",
  "gene_symbol": "CCDC8",
  "term_label": "regulation of mitotic nuclear division"
}